transitive RNA interference [GO:0036453] (biological process) Relationships: is a type of regulatory ncRNA-mediated post-transcriptional gene silencing [GO:0035194] References: PMID:11719187, PMID:12554873, PMID:23724097, PMID:24369430 Sources: GOC:pf Definition: An RNA interference where the silencing signal spreads along the target mRNA in a 5' or 3' direction, outside of the initial target sequence. Also known as: transitive RNAi Subtypes: GO:1990514, GO:1990515